dopamine biosynthetic process from tyrosine [GO:0006585] (biological process) Definition: The chemical reactions and pathways resulting in the formation of dopamine (3,4-dihydroxyphenylethylamine) from L-tyrosine, via the metabolic precursor 3,4-dihydroxy-L-phenylalanine (L-dopa). Dopamine is a catecholamine neurotransmitter and a metabolic precursor of norepinephrine and epinephrine. Sources: GOC:bf, GOC:jl, ISBN:0198506732 Also known as: dopamine anabolism from tyrosine, dopamine formation from tyrosine, dopamine synthesis from tyrosine Relationships: is a type of GO:0006570; is a type of dopamine biosynthetic process [GO:0042416]